negative regulation of retrograde axon cargo transport [GO:2001018] (biological process) Also known as: negative regulation of retrograde axonal transport Subtypes: negative regulation of retrograde dense core granule transport [GO:1901955] Definition: Any process that stops, prevents or reduces the frequency, rate or extent of retrograde axon cargo transport. Sources: GOC:obol Relationships: is a type of negative regulation of intracellular transport [GO:0032387]; is a type of regulation of retrograde axon cargo transport [GO:2001017]; negatively regulates retrograde axonal transport [GO:0008090]